{
  "gene": "UniProtKB:Q15020",
  "gene_name": "Squamous cell carcinoma antigen recognized by T-cells 3",
  "term_id": "GO:0061574",
  "gene_symbol": "SART3",
  "term_label": "ASAP complex"
}